regulation of anterograde axonal transport of mitochondrion [GO:0061880] (biological process) Relationships: is a type of GO:1902513; regulates anterograde axonal transport of mitochondrion [GO:0098957] Subtypes: positive regulation of anterograde axonal transport of mitochondrion [GO:0061881], negative regulation of anterograde axonal transport of mitochondrion [GO:0061882] Definition: Any process that modulates the frequency, rate or extent of the directed movement of mitochondria along microtubules in axons away from the cell body and towards the presynapse. References: PMID:24302729 Also known as: regulation of anterograde axon transport of mitochondria